acetyl-CoA hydrolase activity [GO:0003986] (molecular function) Definition: Catalysis of the reaction: acetyl-CoA + H2O = acetate + CoA + H+. Sources: EC:3.1.2.1, RHEA:20289 Also known as: acetyl coenzyme A acylase activity, acetyl coenzyme A deacylase activity, acetyl coenzyme A hydrolase activity, acetyl-CoA acylase activity, acetyl-CoA deacylase activity, acetyl-CoA thiol esterase activity Relationships: is a type of acyl-CoA hydrolase activity [GO:0016289]